{
  "gene_symbol": "PSEN1",
  "term_label": "membrane protein ectodomain proteolysis",
  "gene": "UniProtKB:P49768",
  "gene_name": "Presenilin-1",
  "term_id": "GO:0006509"
}